negative regulation of T-helper 2 cell differentiation [GO:0045629] (biological process) Note: Note that immunologists typically use the word 'development' to refer to cells of B or T cell lineages undergoing the process that GO describes as 'cell differentiation'. Sources: GOC:go_curators Definition: Any process that stops, prevents, or reduces the frequency, rate or extent of T-helper 2 cell differentiation. Relationships: is a type of negative regulation of type 2 immune response [GO:0002829]; is a type of negative regulation of T-helper cell differentiation [GO:0045623]; is a type of regulation of T-helper 2 cell differentiation [GO:0045628]; negatively regulates T-helper 2 cell differentiation [GO:0045064] Also known as: down regulation of T-helper 2 cell differentiation, down-regulation of T-helper 2 cell differentiation, downregulation of T-helper 2 cell differentiation, inhibition of T-helper 2 cell differentiation, negative regulation of T-helper 2 cell development